{
  "term_label": "chromatin",
  "gene_name": "Testis-specific Y-encoded protein 8",
  "gene_symbol": "TSPY8",
  "term_id": "GO:0000785",
  "gene": "UniProtKB:P0CW00"
}